{
  "term_label": "Unknown biological process",
  "term_id": "UNKNOWN:0002",
  "gene_symbol": "TRBD1",
  "gene_name": "T cell receptor beta diversity 1",
  "gene": "UniProtKB:P0DPI4"
}